{
  "term_id": "GO:0005829",
  "gene_name": "Serine_threonine-protein kinase WNK1",
  "gene_symbol": "WNK1",
  "term_label": "cytosol",
  "gene": "UniProtKB:Q9H4A3"
}